chemokinesis [GO:0042466] (biological process) Definition: A response by a motile cell to a soluble chemical that involves an increase or decrease in speed (positive or negative orthokinesis) or of frequency of movement or a change in the frequency or magnitude of turning behavior (klinokinesis). Regulation: regulated by regulation of chemokinesis [GO:1904365]; negatively regulated by GO:1904366; positively regulated by positive regulation of chemokinesis [GO:1904367] References: PMID:2073411 Sources: GOC:jl Relationships: is a type of kinesis [GO:0042465]